{
  "gene": "UniProtKB:Q01814",
  "term_id": "GO:0005388",
  "term_label": "P-type calcium transporter activity",
  "gene_symbol": "ATP2B2",
  "gene_name": "Plasma membrane calcium-transporting ATPase 2"
}